{
  "gene_name": "Tetra-peptide repeat homeobox protein 1",
  "term_label": "Unknown molecular function",
  "gene_symbol": "TPRX1",
  "term_id": "UNKNOWN:0001",
  "gene": "UniProtKB:Q8N7U7"
}